{
  "term_label": "dendrite morphogenesis",
  "term_id": "GO:0048813",
  "gene_symbol": "BTBD3",
  "gene": "UniProtKB:Q9Y2F9",
  "gene_name": "BTB_POZ domain-containing protein 3"
}